regulation of response to red or far red light [GO:2000030] (biological process) Sources: GOC:obol Relationships: is a type of regulation of response to stimulus [GO:0048583]; regulates response to red or far red light [GO:0009639] Definition: Any process that modulates the frequency, rate or extent of response to red or far red light. Subtypes: regulation of photomorphogenesis [GO:0010099], regulation of red or far-red light signaling pathway [GO:0090227], regulation of shade avoidance [GO:1902446]